protein insertion into ER membrane by stop-transfer membrane-anchor sequence [GO:0045050] (biological process) Sources: ISBN:0716731363 Definition: A process of protein insertion into the endoplasmic reticulum (ER) membrane in which stop-transfer membrane-anchor sequences become an ER membrane spanning helix. Relationships: is a type of protein insertion into ER membrane [GO:0045048] Also known as: protein insertion into ER membrane, stop-transfer membrane-anchor sequence mediated, protein insertion into endoplasmic reticulum membrane by stop-transfer membrane-anchor sequence, protein-ER insertion by stop-transfer membrane-anchor sequence, protein-endoplasmic reticulum insertion by stop-transfer membrane-anchor sequence, stop-transfer membrane-anchor sequence mediated protein insertion into ER membrane